{
  "gene_symbol": "KLK15",
  "term_id": "GO:0051604",
  "term_label": "protein maturation",
  "gene": "UniProtKB:Q9H2R5",
  "gene_name": "Kallikrein-15"
}